{
  "term_label": "immunoglobulin complex",
  "gene": "UniProtKB:A0A075B6S4",
  "gene_symbol": "IGKV1D-17",
  "gene_name": "Immunoglobulin kappa variable 1D-17",
  "term_id": "GO:0019814"
}